L-ornithine catabolic process, by decarboxylation [GO:0019467] (biological process) Definition: The chemical reactions and pathways resulting in the breakdown of L-ornithine by decarboxylation. Sources: GOC:go_curators Relationships: is_a GO:0006593; has part carboxy-lyase activity [GO:0016831] Also known as: ornithine breakdown, by decarboxylation, ornithine degradation, by decarboxylation